cellular response to mineralocorticoid stimulus [GO:0071389] (biological process) Definition: Any process that results in a change in state or activity of a cell (in terms of movement, secretion, enzyme production, gene expression, etc.) as a result of a mineralocorticoid stimulus. Mineralocorticoids are hormonal C21 corticosteroids synthesized from cholesterol and characterized by their similarity to aldosterone. Mineralocorticoids act primarily on water and electrolyte balance. Relationships: is a type of response to mineralocorticoid [GO:0051385]; is a type of GO:0071384 Subtypes: cellular response to corticosterone stimulus [GO:0071386], cellular response to 11-deoxycorticosterone [GO:1903497], GO:1904045 Sources: GOC:mah